{
  "gene": "UniProtKB:Q3C1V8",
  "term_label": "regulation of transcription by RNA polymerase II",
  "term_id": "GO:0006357",
  "gene_symbol": "BSX",
  "gene_name": "Brain-specific homeobox protein homolog"
}